{
  "term_id": "GO:0015671",
  "gene": "UniProtKB:P69891",
  "gene_symbol": "HBG1",
  "gene_name": "Hemoglobin subunit gamma-1",
  "term_label": "oxygen transport"
}